{
  "gene_name": "Vesicular inhibitory amino acid transporter",
  "term_id": "GO:0030672",
  "gene_symbol": "SLC32A1",
  "gene": "UniProtKB:Q9H598",
  "term_label": "synaptic vesicle membrane"
}